anisotropic cell growth [GO:0051211] (biological process) Also known as: non-isotropic cell growth Sources: GOC:ai Definition: The process in which a cell irreversibly increases in size in one or more axes, where the growth rate varies according to the direction of growth. Growth may be limited to a particular axis, axes, or to particular locations on the surface of the cell. Relationships: is a type of cell growth [GO:0016049]